{
  "term_label": "regulation of transcription by RNA polymerase II",
  "gene_name": "Zinc finger protein 597",
  "term_id": "GO:0006357",
  "gene_symbol": "ZNF597",
  "gene": "UniProtKB:Q96LX8"
}